protein deglycosylation involved in glycoprotein catabolic process [GO:0035977] (biological process) Subtypes: mannose trimming involved in glycoprotein ERAD pathway [GO:1904382] Relationships: is a type of protein deglycosylation [GO:0006517]; is part of glycoprotein catabolic process [GO:0006516] Definition: The removal of sugar residues from a glycosylated protein that contributes to the breakdown of a glycoprotein. Sources: GOC:bf, GOC:vw